{
  "gene": "UniProtKB:P42677",
  "gene_symbol": "RPS27",
  "gene_name": "Small ribosomal subunit protein eS27",
  "term_label": "ribosomal small subunit assembly",
  "term_id": "GO:0000028"
}